{
  "gene": "UniProtKB:O75290",
  "term_label": "regulation of transcription by RNA polymerase II",
  "term_id": "GO:0006357",
  "gene_symbol": "ZNF780A",
  "gene_name": "Zinc finger protein 780A"
}